{
  "gene_name": "Rho guanine nucleotide exchange factor 33",
  "gene_symbol": "ARHGEF33",
  "gene": "UniProtKB:A8MVX0",
  "term_id": "UNKNOWN:0003",
  "term_label": "Unknown cellular component"
}